stomatal closure [GO:0090332] (biological process) Definition: The process of closing of stomata, pores in the epidermis of leaves and stems bordered by two guard cells and serving in gas exchange. Regulation: regulated by regulation of stomatal closure [GO:0090333] Relationships: is a type of stomatal movement [GO:0010118] Sources: GOC:tb